ecgonone methyl ester biosynthetic process [GO:1901872] (biological process) References: PMID:22665766 Sources: GOC:TermGenie Also known as: ecgonone methyl ester anabolism, ecgonone methyl ester biosynthesis, ecgonone methyl ester formation, ecgonone methyl ester synthesis Definition: The chemical reactions and pathways resulting in the formation of ecgonone methyl ester. Relationships: is a type of GO:0009710; is a type of GO:0042181